propanoyl-CoA C-acyltransferase activity [GO:0033814] (MF) Sources: RHEA:16865 Definition: Catalysis of the reaction: choloyl-CoA + propanoyl-CoA = 3alpha,7alpha,12alpha-trihydroxy-24-oxo-5beta-cholestan-26-oyl-CoA + CoA. Relationships: is a type of C-acyltransferase activity [GO:0016408] Also known as: peroxisomal thiolase 2 activity, 3alpha,7alpha,12alpha-trihydroxy-5beta-cholanoyl-CoA:propanoyl-CoA C-acyltransferase activity, PTE-2, SCP-X, SCPchi, sterol carrier protein-X, sterol carrier protein-chi